dCDP catabolic process [GO:0006251] (biological process) Relationships: is a type of pyrimidine deoxyribonucleoside diphosphate catabolic process [GO:0009198]; is a type of pyrimidine deoxyribonucleotide catabolic process [GO:0009223]; is a type of dCDP metabolic process [GO:0046062] Sources: ISBN:0198506732 Also known as: dCDP breakdown, dCDP catabolism, dCDP degradation Definition: The chemical reactions and pathways resulting in the breakdown of dCDP, deoxycytidine 5'-diphosphate.